{
  "gene_name": "Phosphoglycerate mutase 1",
  "term_label": "cytosol",
  "gene_symbol": "PGAM1",
  "term_id": "GO:0005829",
  "gene": "UniProtKB:P18669"
}